{
  "gene": "UniProtKB:Q86TB3",
  "term_id": "UNKNOWN:0001",
  "gene_symbol": "ALPK2",
  "gene_name": "Alpha-protein kinase 2",
  "term_label": "Unknown molecular function"
}